myosin II filament disassembly [GO:0031037] (biological process) Relationships: is a type of myosin filament disassembly [GO:0031035]; is a type of GO:0031038 Definition: The disassembly of a bipolar filament composed of myosin II molecules. Regulation: regulated by GO:0043521 Sources: GOC:mah Also known as: myosin II depolymerization